nucleolus-associated heterochromatin [GO:0097424] (cellular component) Sources: NIF_Subcellular:sao1210952635 Definition: Dense particles of heterochromatin, consisting of a loosely twisted strand about 600 Angstrom thick, found associated with the nucleolus. Relationships: is a type of nucleolar chromatin [GO:0030874]